{
  "term_id": "GO:0000165",
  "term_label": "MAPK cascade",
  "gene_name": "Dual specificity mitogen-activated protein kinase kinase 6",
  "gene": "UniProtKB:P52564",
  "gene_symbol": "MAP2K6"
}